{
  "gene_name": "Triple functional domain protein",
  "term_label": "guanyl-nucleotide exchange factor activity",
  "term_id": "GO:0005085",
  "gene": "UniProtKB:O75962",
  "gene_symbol": "TRIO"
}